{
  "term_label": "Unknown cellular component",
  "term_id": "UNKNOWN:0003",
  "gene_name": "Putative UPF0633 protein ENSP00000303136",
  "gene": "UniProtKB:Q5VV11",
  "gene_symbol": "Q5VV11"
}